{
  "term_id": "GO:0030136",
  "term_label": "clathrin-coated vesicle",
  "gene_name": "HCLS1-associated protein X-1",
  "gene": "UniProtKB:O00165",
  "gene_symbol": "HAX1"
}